{
  "gene": "UniProtKB:P26196",
  "term_id": "GO:0034063",
  "gene_symbol": "DDX6",
  "term_label": "stress granule assembly",
  "gene_name": "Probable ATP-dependent RNA helicase DDX6"
}